G-protein beta/gamma-subunit complex binding [GO:0031683] (molecular function) Relationships: is a type of protein-containing complex binding [GO:0044877] Sources: GOC:nln, GOC:vw Definition: Binding to a complex of G-protein beta/gamma subunits.